{
  "term_id": "GO:0051539",
  "term_label": "4 iron, 4 sulfur cluster binding",
  "gene_symbol": "RSAD1",
  "gene": "UniProtKB:Q9HA92",
  "gene_name": "Radical S-adenosyl methionine domain-containing protein 1, mitochondrial"
}